{
  "gene": "UniProtKB:O43488",
  "gene_name": "Aflatoxin B1 aldehyde reductase member 2",
  "term_id": "UNKNOWN:0002",
  "term_label": "Unknown biological process",
  "gene_symbol": "AKR7A2"
}